{
  "gene_name": "cTAGE family member 8",
  "term_id": "GO:0006888",
  "gene": "UniProtKB:P0CG41",
  "gene_symbol": "CTAGE8",
  "term_label": "endoplasmic reticulum to Golgi vesicle-mediated transport"
}